{
  "term_label": "eukaryotic translation initiation factor 2 complex",
  "gene_name": "Eukaryotic translation initiation factor 2A",
  "gene_symbol": "EIF2A",
  "term_id": "GO:0005850",
  "gene": "UniProtKB:Q9BY44"
}